urogenital system development [GO:0001655] (biological process) Definition: The process whose specific outcome is the progression of the urogenital system over time, from its formation to the mature structure. Relationships: is a type of system development [GO:0048731]; has part renal system development [GO:0072001] Sources: GOC:go_curators